{
  "gene": "UniProtKB:Q6ZN84",
  "term_label": "Unknown molecular function",
  "gene_symbol": "CCDC81",
  "gene_name": "Coiled-coil domain-containing protein 81",
  "term_id": "UNKNOWN:0001"
}